{
  "term_id": "GO:0042758",
  "gene": "UniProtKB:P28330",
  "gene_symbol": "ACADL",
  "gene_name": "Long-chain specific acyl-CoA dehydrogenase, mitochondrial",
  "term_label": "long-chain fatty acid catabolic process"
}